{
  "gene_name": "Olfactory receptor 9G4",
  "term_label": "Unknown cellular component",
  "gene": "UniProtKB:Q8NGQ1",
  "term_id": "UNKNOWN:0003",
  "gene_symbol": "OR9G4"
}